{
  "gene": "UniProtKB:Q8WUY3",
  "term_label": "Unknown molecular function",
  "gene_name": "Protein prune homolog 2",
  "term_id": "UNKNOWN:0001",
  "gene_symbol": "PRUNE2"
}